acyl-CoA dehydrogenase activity [GO:0003995] (molecular function) Definition: Catalysis of the reaction: a 2,3-saturated acyl-CoA + H+ oxidized [electron-transfer flavoprotein] = a (2E)-enoyl-CoA + reduced [electron-transfer flavoprotein]. Also known as: acyl CoA dehydrogenase activity, acyl coenzyme A dehydrogenase activity, acyl-CoA reductase activity, fatty acyl coenzyme A dehydrogenase activity, fatty-acyl-CoA dehydrogenase activity, general acyl CoA dehydrogenase activity Subtypes: glutaryl-CoA dehydrogenase activity [GO:0004361], long-chain fatty acyl-CoA dehydrogenase activity [GO:0004466], short-chain fatty acyl-CoA dehydrogenase activity [GO:0016937], very-long-chain fatty acyl-CoA dehydrogenase activity [GO:0017099], GO:0070991 Relationships: is a type of GO:0052890 Sources: RHEA:44704